gamma-aminobutyric acid signaling pathway [GO:0007214] (biological process) Relationships: is a type of cell-cell signaling [GO:0007267]; has part GABA receptor activity [GO:0016917] Also known as: 4-aminobutanoate signaling pathway, 4-aminobutanoate signalling pathway, 4-aminobutyrate signaling pathway, 4-aminobutyrate signalling pathway, GABA signaling pathway, GABA signalling pathway, gamma-aminobutyric acid signalling pathway Sources: GOC:mah Subtypes: GO:0160001 Definition: The series of molecular signals generated by the binding of gamma-aminobutyric acid (GABA, 4-aminobutyrate), an amino acid which acts as a neurotransmitter in some organisms, to its receptor on the surface of a target cell.